{
  "gene": "UniProtKB:Q8IWI9",
  "gene_name": "MAX gene-associated protein",
  "term_id": "GO:0001708",
  "term_label": "cell fate specification",
  "gene_symbol": "MGA"
}